{
  "gene": "UniProtKB:Q9Y2V2",
  "term_id": "GO:0005737",
  "gene_symbol": "CARHSP1",
  "term_label": "cytoplasm",
  "gene_name": "Calcium-regulated heat-stable protein 1"
}